{
  "term_label": "plasma membrane",
  "gene": "UniProtKB:A8MXK1",
  "gene_name": "V-set and transmembrane domain-containing protein 5",
  "gene_symbol": "VSTM5",
  "term_id": "GO:0005886"
}